{
  "term_id": "GO:0035686",
  "term_label": "sperm fibrous sheath",
  "gene": "UniProtKB:O75952",
  "gene_symbol": "CABYR",
  "gene_name": "Calcium-binding tyrosine phosphorylation-regulated protein"
}